{
  "term_id": "GO:0006363",
  "gene_symbol": "CAVIN1",
  "term_label": "termination of RNA polymerase I transcription",
  "gene": "UniProtKB:Q6NZI2",
  "gene_name": "Caveolae-associated protein 1"
}